{
  "term_id": "GO:0038023",
  "gene_name": "Integrin alpha-3",
  "gene": "UniProtKB:P26006",
  "term_label": "signaling receptor activity",
  "gene_symbol": "ITGA3"
}